{
  "term_id": "UNKNOWN:0003",
  "gene_symbol": "FAM13C",
  "term_label": "Unknown cellular component",
  "gene": "UniProtKB:Q8NE31",
  "gene_name": "Protein FAM13C"
}